{
  "gene_symbol": "ROCK1",
  "term_label": "Rho protein signal transduction",
  "gene": "UniProtKB:Q13464",
  "gene_name": "Rho-associated protein kinase 1",
  "term_id": "GO:0007266"
}